{
  "term_label": "negative regulation of G1/S transition of mitotic cell cycle",
  "term_id": "GO:2000134",
  "gene": "UniProtKB:Q08999",
  "gene_symbol": "RBL2",
  "gene_name": "Retinoblastoma-like protein 2"
}